synaptic vesicle targeting [GO:0016080] (BP) Definition: The process in which synaptic vesicles are directed to specific destination membranes, mediated by molecules at the vesicle membrane and target membrane surfaces. Sources: GOC:mah Relationships: is a type of GO:0006903; is a type of GO:0140029; is part of GO:0016079